(1->6)-beta-D-glucan catabolic process [GO:0006079] (biological process) Sources: GOC:ai Also known as: 1,6-beta-D-glucan breakdown, 1,6-beta-D-glucan catabolic process, 1,6-beta-D-glucan catabolism, 1,6-beta-D-glucan degradation, beta-1,6 glucan breakdown, beta-1,6 glucan catabolic process, beta-1,6 glucan catabolism, beta-1,6 glucan degradation Definition: The chemical reactions and pathways resulting in the breakdown of (1->6)-beta-D-glucans. Relationships: is a type of (1->6)-beta-D-glucan metabolic process [GO:0006077]; is a type of beta-glucan catabolic process [GO:0051275]